{
  "term_id": "GO:0006357",
  "term_label": "regulation of transcription by RNA polymerase II",
  "gene_name": "Zinc finger protein 391",
  "gene": "UniProtKB:Q9UJN7",
  "gene_symbol": "ZNF391"
}